{
  "gene_symbol": "IDO1",
  "gene": "UniProtKB:P14902",
  "term_id": "GO:0004833",
  "gene_name": "Indoleamine 2,3-dioxygenase 1",
  "term_label": "L-tryptophan 2,3-dioxygenase activity"
}